{
  "gene_symbol": "XBP1",
  "gene": "UniProtKB:P17861",
  "term_label": "DNA-binding transcription factor activity, RNA polymerase II-specific",
  "term_id": "GO:0000981",
  "gene_name": "X-box-binding protein 1"
}